response to plumbagin [GO:1902708] (BP) Subtypes: GO:1902709 Definition: Any process that results in a change in state or activity of a cell or an organism (in terms of movement, secretion, enzyme production, gene expression, etc.) as a result of a plumbagin stimulus. Relationships: is a type of response to ketone [GO:1901654] References: PMID:23028742 Sources: GOC:TermGenie, GO_REF:0000071